{
  "term_id": "GO:0005737",
  "gene_symbol": "C15orf40",
  "gene": "UniProtKB:Q8WUR7",
  "gene_name": "UPF0235 protein C15orf40",
  "term_label": "cytoplasm"
}